positive regulation of teliospore formation [GO:0075257] (biological process) Sources: GOC:pamgo_curators Relationships: is a type of positive regulation of asexual sporulation resulting in formation of a cellular spore [GO:0043945]; is a type of GO:0075256; positively regulates teliospore formation [GO:0075255] Definition: Any process that activates, maintains or increases the frequency, rate or extent of teliospore formation, which is the formation of a thick-walled resting or overwintering spore produced by the rust fungi (Uredinales) and smut fungi (Ustilaginales) in which karyogamy occurs.